{
  "gene": "UniProtKB:Q9NP94",
  "term_label": "zinc ion transmembrane transport",
  "gene_name": "Zinc transporter ZIP2",
  "gene_symbol": "SLC39A2",
  "term_id": "GO:0071577"
}